{
  "gene_name": "CTTNBP2 N-terminal-like protein",
  "gene_symbol": "CTTNBP2NL",
  "term_id": "UNKNOWN:0001",
  "term_label": "Unknown molecular function",
  "gene": "UniProtKB:Q9P2B4"
}